{
  "term_label": "Golgi membrane",
  "gene_name": "N-acetylneuraminate 9-O-acetyltransferase",
  "term_id": "GO:0000139",
  "gene": "UniProtKB:Q96PB1",
  "gene_symbol": "CASD1"
}